response to nitric oxide [GO:0071731] (biological process) Relationships: is a type of GO:1901698; is a type of GO:1901700 Definition: Any process that results in a change in state or activity of a cell or an organism (in terms of movement, secretion, enzyme production, gene expression, etc.) as a result of a nitric oxide stimulus. Subtypes: cellular response to nitric oxide [GO:0071732] Sources: GOC:mah, GOC:yaf